{
  "gene": "UniProtKB:Q86US8",
  "gene_name": "Telomerase-binding protein EST1A",
  "term_label": "nuclear-transcribed mRNA catabolic process, nonsense-mediated decay",
  "gene_symbol": "SMG6",
  "term_id": "GO:0000184"
}